diol metabolic process [GO:0034311] (biological process) Also known as: diol metabolism, dihydric alcohol metabolic process Relationships: is_a polyol metabolic process [GO:0019751] Definition: The chemical reactions and pathways involving a diol, a compound that contains two hydroxy groups, generally assumed to be, but not necessarily, alcoholic. Sources: GOC:curators Subtypes: GO:0006667, sphingosine metabolic process [GO:0006670], diol biosynthetic process [GO:0034312], GO:0034313, GO:0042844, tetrahydrobiopterin metabolic process [GO:0046146]